{
  "term_label": "negative regulation of transcription by RNA polymerase II",
  "gene_symbol": "ATXN1L",
  "gene_name": "Ataxin-1-like",
  "gene": "UniProtKB:P0C7T5",
  "term_id": "GO:0000122"
}